{
  "gene_symbol": "METAP2",
  "term_id": "GO:0005737",
  "gene": "UniProtKB:P50579",
  "gene_name": "Methionine aminopeptidase 2",
  "term_label": "cytoplasm"
}